regulation of macroautophagy [GO:0016241] (biological process) Sources: GOC:krc Subtypes: positive regulation of macroautophagy [GO:0016239], negative regulation of macroautophagy [GO:0016242], regulation of reticulophagy [GO:0140500], regulation of autophagosome maturation [GO:1901096], regulation of mitophagy [GO:1901524], regulation of xenophagy [GO:1904415], GO:1904502, GO:1905335 Also known as: regulation of starvation-induced autophagy Relationships: is a type of regulation of autophagy [GO:0010506]; regulates macroautophagy [GO:0016236] Definition: Any process that modulates the frequency, rate or extent of macroautophagy.